{
  "term_label": "Unknown molecular function",
  "gene": "UniProtKB:A0A1B0GTR4",
  "gene_symbol": "SPRR5",
  "term_id": "UNKNOWN:0001",
  "gene_name": "Putative small proline-rich protein 5"
}